{
  "term_id": "GO:0005615",
  "term_label": "extracellular space",
  "gene": "UniProtKB:P29622",
  "gene_name": "Kallistatin",
  "gene_symbol": "SERPINA4"
}